{
  "gene_symbol": "TLR10",
  "gene": "UniProtKB:Q9BXR5",
  "term_label": "Toll-like receptor 2 binding",
  "gene_name": "Toll-like receptor 10",
  "term_id": "GO:0035663"
}